silicon efflux transmembrane transporter activity [GO:0032523] (molecular function) Relationships: is a type of monoatomic cation transmembrane transporter activity [GO:0008324]; is a type of efflux transmembrane transporter activity [GO:0015562] References: PMID:17625566 Sources: GOC:mah Also known as: silicon efflux transporter activity Definition: Enables the transfer of silicon from the inside of the cell to the outside of the cell across a membrane.